{
  "gene_symbol": "TFDP1",
  "term_label": "RNA polymerase II transcription regulatory region sequence-specific DNA binding",
  "gene": "UniProtKB:Q14186",
  "gene_name": "Transcription factor Dp-1",
  "term_id": "GO:0000977"
}